{
  "term_label": "glutathione metabolic process",
  "term_id": "GO:0006749",
  "gene_name": "Glutathione S-transferase P",
  "gene_symbol": "GSTP1",
  "gene": "UniProtKB:P09211"
}